tangential migration from the subventricular zone to the olfactory bulb [GO:0022028] (biological process) Also known as: rostral migratory stream migration Relationships: is a type of GO:0022029; BFO_0000050 olfactory bulb development [GO:0021772] Sources: GOC:cls, GOC:dgh, GOC:dph, GOC:jid, GO_REF:0000021 Subtypes: postnatal olfactory bulb interneuron migration [GO:0021827], embryonic olfactory bulb interneuron precursor migration [GO:0021831] Definition: The migration of cells in the telencephalon from the subventricular zone to the olfactory bulb in which cells move orthogonally to the direction of radial migration and do not use radial glial cell processes as substrates for migration.